{
  "term_label": "Unknown molecular function",
  "term_id": "UNKNOWN:0001",
  "gene": "UniProtKB:O75379",
  "gene_symbol": "VAMP4",
  "gene_name": "Vesicle-associated membrane protein 4"
}